{
  "gene_name": "Rho-related GTP-binding protein RhoN",
  "gene_symbol": "RND2",
  "term_label": "GTPase activity",
  "term_id": "GO:0003924",
  "gene": "UniProtKB:P52198"
}